5'-3' RNA helicase activity [GO:0032574] (molecular function) Relationships: is a type of RNA helicase activity [GO:0003724] Definition: Unwinding of an RNA helix in the 5' to 3' direction, driven by ATP hydrolysis. Also known as: 5' to 3' RNA helicase activity, ATP-dependent 5' to 3' RNA helicase activity, ATP-dependent 5'-3' RNA helicase activity Sources: GOC:jp